{
  "term_id": "GO:0007052",
  "gene_symbol": "BIRC5",
  "gene": "UniProtKB:O15392",
  "term_label": "mitotic spindle organization",
  "gene_name": "Baculoviral IAP repeat-containing protein 5"
}